{
  "gene": "UniProtKB:Q4VXF1",
  "gene_name": "Putative protein FAM74A3",
  "term_id": "UNKNOWN:0001",
  "term_label": "Unknown molecular function",
  "gene_symbol": "FAM74A3"
}